{
  "term_label": "calcium ion homeostasis",
  "gene_symbol": "CIB3",
  "gene_name": "Calcium and integrin-binding family member 3",
  "gene": "UniProtKB:Q96Q77",
  "term_id": "GO:0055074"
}